{
  "term_id": "GO:0016538",
  "gene_symbol": "CCNJL",
  "gene": "UniProtKB:Q8IV13",
  "term_label": "cyclin-dependent protein serine/threonine kinase regulator activity",
  "gene_name": "Cyclin-J-like protein"
}